{
  "gene_name": "Ubiquitin-conjugating enzyme E2 E1",
  "term_label": "ubiquitin conjugating enzyme activity",
  "gene_symbol": "UBE2E1",
  "term_id": "GO:0061631",
  "gene": "UniProtKB:P51965"
}